negative regulation of acute inflammatory response to antigenic stimulus [GO:0002865] (biological process) Sources: GOC:add Subtypes: negative regulation of hypersensitivity [GO:0002884] Also known as: down regulation of acute inflammatory response to antigenic stimulus, down-regulation of acute inflammatory response to antigenic stimulus, downregulation of acute inflammatory response to antigenic stimulus, inhibition of acute inflammatory response to antigenic stimulus Definition: Any process that stops, prevents, or reduces the frequency, rate, or extent of an acute inflammatory response to an antigenic stimulus. Relationships: is a type of negative regulation of acute inflammatory response [GO:0002674]; is a type of negative regulation of inflammatory response to antigenic stimulus [GO:0002862]; is a type of regulation of acute inflammatory response to antigenic stimulus [GO:0002864]; negatively regulates acute inflammatory response to antigenic stimulus [GO:0002438]